{
  "gene": "UniProtKB:Q6NXG1",
  "gene_name": "Epithelial splicing regulatory protein 1",
  "term_id": "GO:0043484",
  "gene_symbol": "ESRP1",
  "term_label": "regulation of RNA splicing"
}